protein localization to mast cell secretory granule [GO:0033367] (biological process) Relationships: is a type of protein localization to secretory granule [GO:0033366]; is part of mast cell secretory granule organization [GO:0033364] Subtypes: GO:0033368 Also known as: protein localisation in mast cell secretory granule, protein localization in mast cell secretory granule Sources: GOC:mah Definition: A process in which a protein is transported to, or maintained in, a location within a secretory granule in a mast cell.